Sm-like protein family complex [GO:0120114] (cellular component) References: PMID:19121818, PMID:27627834 Sources: GOC:bhm, GOC:krc Subtypes: small nuclear ribonucleoprotein complex [GO:0030532], GO:0032797, pICln-Sm protein complex [GO:0034715], SMN-Gemin2 complex [GO:0034718], SMN-Sm protein complex [GO:0034719], GO:0120115, Lsm1-7-Pat1 complex [GO:1990726] Relationships: is_a protein-containing complex [GO:0032991] Definition: A protein complex containing members of the Like-Sm family of proteins, which includes both the Sm proteins and the Lsm proteins, and which generally form hexameric or heptameric ring structures which bind to RNA. While some of these ring complexes may form independently of RNA, many only form in association with their target RNA. In addition to Lsm-family proteins, many of these complexes contain additional protein members. Members of this family of complexes include the snRNPs which comprise the majority of the spliceosome. Others are involved in the 5' to 3' degradation pathways of mRNAs in the cytoplasm and of unspliced transcripts in the nucleus, as well as other diverse roles.